{
  "gene": "UniProtKB:P12643",
  "gene_name": "Bone morphogenetic protein 2",
  "term_label": "heart morphogenesis",
  "term_id": "GO:0003007",
  "gene_symbol": "BMP2"
}